{
  "gene_symbol": "UNC13C",
  "term_label": "plasma membrane",
  "term_id": "GO:0005886",
  "gene": "UniProtKB:Q8NB66",
  "gene_name": "Protein unc-13 homolog C"
}